response to karrikin [GO:0080167] (biological process) Definition: Any process that results in a change in state or activity of a cell or an organism (in terms of movement, secretion, enzyme production, gene expression, etc.) as a result of a karrikin stimulus. Karrikins are signaling molecules in smoke from burning vegetation that trigger seed germination for many angiosperms (flowering plants). References: PMID:20351290 Relationships: is_a response to abiotic stimulus [GO:0009628]